{
  "gene_name": "Pre-mRNA-splicing factor RBM22",
  "gene": "UniProtKB:Q9NW64",
  "term_id": "GO:0000974",
  "gene_symbol": "RBM22",
  "term_label": "Prp19 complex"
}